{
  "term_label": "Unknown cellular component",
  "gene_name": "Hexosaminidase D",
  "gene_symbol": "HEXD",
  "gene": "UniProtKB:Q8WVB3",
  "term_id": "UNKNOWN:0003"
}